{
  "gene_name": "Golgi pH regulator B",
  "term_label": "Golgi cisterna membrane",
  "gene": "UniProtKB:P0CG08",
  "gene_symbol": "GPR89B",
  "term_id": "GO:0032580"
}